{
  "term_label": "cytosol",
  "term_id": "GO:0005829",
  "gene_symbol": "USP17L4",
  "gene_name": "Inactive ubiquitin carboxyl-terminal hydrolase 17-like protein 4",
  "gene": "UniProtKB:A6NCW7"
}